regulation by virus of viral protein levels in host cell [GO:0046719] (biological process) Definition: Any virus-mediated process that modulates the levels of viral proteins in a cell. Relationships: is a type of regulation of viral process [GO:0050792]; is a type of regulation of biological quality [GO:0065008] Also known as: regulation of viral protein levels Sources: GOC:ai Subtypes: negative regulation by virus of viral protein levels in host cell [GO:0046725], positive regulation by virus of viral protein levels in host cell [GO:0046726]